{
  "term_id": "GO:0006357",
  "gene": "UniProtKB:Q8N184",
  "gene_name": "Zinc finger protein 567",
  "gene_symbol": "ZNF567",
  "term_label": "regulation of transcription by RNA polymerase II"
}